{
  "term_label": "DNA-binding transcription factor activity, RNA polymerase II-specific",
  "gene": "UniProtKB:P17027",
  "term_id": "GO:0000981",
  "gene_symbol": "ZNF23",
  "gene_name": "Zinc finger protein 23"
}